{
  "gene": "UniProtKB:Q9NX18",
  "term_id": "GO:0006099",
  "gene_name": "Succinate dehydrogenase assembly factor 2, mitochondrial",
  "gene_symbol": "SDHAF2",
  "term_label": "tricarboxylic acid cycle"
}